{
  "term_id": "GO:0005634",
  "gene_name": "Histone H2B type W-T",
  "gene": "UniProtKB:Q7Z2G1",
  "term_label": "nucleus",
  "gene_symbol": "H2BW1"
}